{
  "term_id": "GO:0005212",
  "gene_symbol": "CRYBG3",
  "gene_name": "Very large A-kinase anchor protein",
  "gene": "UniProtKB:Q68DQ2",
  "term_label": "structural constituent of eye lens"
}